salutaridinol 7-O-acetyltransferase activity [GO:0047180] (molecular function) Sources: EC:2.3.1.150, RHEA:22856 Relationships: is a type of O-acetyltransferase activity [GO:0016413] Definition: Catalysis of the reaction: (7S)-salutaridinol + acetyl-CoA = (7S)-O-acetylsalutaridinol + CoA. Also known as: acetyl-CoA:salutaridinol 7-O-acetyltransferase activity